medial cortex [GO:0031097] (cellular component) References: PMID:15572668, PMID:19474789 Sources: GOC:vw Also known as: medial ring Relationships: is a type of GO:0099738; is part of cell division site [GO:0032153] Definition: A medial cortical band overlaying the nucleus which acts as a landmark for contractile ring positioning and plays a role in cell cycle regulation.